{
  "term_label": "ribonucleoprotein complex",
  "gene_name": "Polyadenylate-binding protein 1-like",
  "gene_symbol": "PABPC1L",
  "gene": "UniProtKB:Q4VXU2",
  "term_id": "GO:1990904"
}